{
  "gene_symbol": "CNOT8",
  "term_label": "nuclear-transcribed mRNA catabolic process, deadenylation-dependent decay",
  "gene_name": "CCR4-NOT transcription complex subunit 8",
  "gene": "UniProtKB:Q9UFF9",
  "term_id": "GO:0000288"
}